{
  "term_id": "GO:0005789",
  "gene_symbol": "LMF2",
  "term_label": "endoplasmic reticulum membrane",
  "gene": "UniProtKB:Q9BU23",
  "gene_name": "Lipase maturation factor 2"
}